{
  "gene_name": "DDB1- and CUL4-associated factor 15",
  "term_label": "Unknown molecular function",
  "gene_symbol": "DCAF15",
  "term_id": "UNKNOWN:0001",
  "gene": "UniProtKB:Q66K64"
}